{
  "term_id": "GO:0004459",
  "gene_symbol": "LDHC",
  "term_label": "L-lactate dehydrogenase (NAD+) activity",
  "gene_name": "L-lactate dehydrogenase C chain",
  "gene": "UniProtKB:P07864"
}